{
  "gene": "UniProtKB:Q96DZ5",
  "term_id": "GO:0005938",
  "term_label": "cell cortex",
  "gene_symbol": "CLIP3",
  "gene_name": "CAP-Gly domain-containing linker protein 3"
}